{
  "term_label": "nucleus",
  "gene_name": "Zinc finger protein 470",
  "term_id": "GO:0005634",
  "gene": "UniProtKB:Q6ECI4",
  "gene_symbol": "ZNF470"
}